{
  "gene": "UniProtKB:P52945",
  "gene_name": "Pancreas_duodenum homeobox protein 1",
  "term_id": "GO:0000978",
  "gene_symbol": "PDX1",
  "term_label": "RNA polymerase II cis-regulatory region sequence-specific DNA binding"
}